{
  "gene_name": "Zinc finger protein 627",
  "term_id": "GO:0006357",
  "gene_symbol": "ZNF627",
  "gene": "UniProtKB:Q7L945",
  "term_label": "regulation of transcription by RNA polymerase II"
}